{
  "term_label": "transmembrane transporter activity",
  "gene": "UniProtKB:Q96NT5",
  "gene_name": "Proton-coupled folate transporter",
  "gene_symbol": "SLC46A1",
  "term_id": "GO:0022857"
}